{
  "term_label": "peroxisome organization",
  "gene_name": "Peroxisomal membrane protein PEX16",
  "gene": "UniProtKB:Q9Y5Y5",
  "gene_symbol": "PEX16",
  "term_id": "GO:0007031"
}